{
  "gene": "UniProtKB:Q9H4G0",
  "term_id": "GO:0005886",
  "gene_name": "Band 4.1-like protein 1",
  "gene_symbol": "EPB41L1",
  "term_label": "plasma membrane"
}